{
  "term_id": "GO:0043195",
  "gene_name": "Beta-soluble NSF attachment protein",
  "term_label": "terminal bouton",
  "gene": "UniProtKB:Q9H115",
  "gene_symbol": "NAPB"
}